{
  "gene": "UniProtKB:P15822",
  "term_id": "GO:0000978",
  "gene_symbol": "HIVEP1",
  "gene_name": "Zinc finger protein 40",
  "term_label": "RNA polymerase II cis-regulatory region sequence-specific DNA binding"
}